snRNA localization to Cajal body [GO:0061016] (biological process) Sources: GOC:ascb_2009, GOC:dph, GOC:tb Definition: The directed movement of snRNA, small nuclear ribonucleic acid, to a Cajal body. Relationships: is a type of RNA localization to Cajal body [GO:0090670]